{
  "term_label": "phosphatidylinositol bisphosphate binding",
  "gene_symbol": "CLVS2",
  "gene": "UniProtKB:Q5SYC1",
  "gene_name": "Clavesin-2",
  "term_id": "GO:1902936"
}